{
  "term_id": "GO:0007165",
  "term_label": "signal transduction",
  "gene_name": "Rho-related GTP-binding protein RhoJ",
  "gene": "UniProtKB:Q9H4E5",
  "gene_symbol": "RHOJ"
}